bicarbonate transmembrane transporter activity [GO:0015106] (molecular function) Relationships: is a type of GO:0022857; is part of bicarbonate transport [GO:0015701] Also known as: hydrogencarbonate transmembrane transporter activity Subtypes: sulfate:bicarbonate antiporter activity [GO:0015383], monoatomic cation:bicarbonate symporter activity [GO:0140410], GO:0140829, bicarbonate channel activity [GO:0160133] Definition: Enables the transfer of bicarbonate from one side of a membrane to the other. Bicarbonate is the hydrogencarbonate ion, HCO3-. Sources: GOC:ai